{
  "gene_name": "TBC1 domain family member 31",
  "gene_symbol": "TBC1D31",
  "gene": "UniProtKB:Q96DN5",
  "term_id": "GO:0036064",
  "term_label": "ciliary basal body"
}